{
  "gene_name": "Mas-related G-protein coupled receptor member X1",
  "gene_symbol": "MRGPRX1",
  "term_id": "GO:0004930",
  "gene": "UniProtKB:Q96LB2",
  "term_label": "G protein-coupled receptor activity"
}